{
  "term_label": "entrainment of circadian clock by photoperiod",
  "gene_symbol": "CRY2",
  "gene_name": "Cryptochrome-2",
  "term_id": "GO:0043153",
  "gene": "UniProtKB:Q49AN0"
}